{
  "gene_symbol": "LUZP2",
  "gene_name": "Leucine zipper protein 2",
  "term_label": "Unknown cellular component",
  "term_id": "UNKNOWN:0003",
  "gene": "UniProtKB:Q86TE4"
}